{
  "gene_symbol": "IDI1",
  "term_label": "cytoplasm",
  "term_id": "GO:0005737",
  "gene": "UniProtKB:Q13907",
  "gene_name": "Isopentenyl-diphosphate Delta-isomerase 1"
}